{
  "gene": "UniProtKB:P38935",
  "term_id": "GO:0005634",
  "term_label": "nucleus",
  "gene_name": "DNA-binding protein SMUBP-2",
  "gene_symbol": "IGHMBP2"
}